{
  "term_id": "GO:0005125",
  "gene_symbol": "GDF2",
  "gene": "UniProtKB:Q9UK05",
  "gene_name": "Growth_differentiation factor 2",
  "term_label": "cytokine activity"
}